{
  "gene_name": "Zinc finger protein 519",
  "gene": "UniProtKB:Q8TB69",
  "gene_symbol": "ZNF519",
  "term_label": "regulation of DNA-templated transcription",
  "term_id": "GO:0006355"
}